{
  "term_label": "Unknown cellular component",
  "gene_name": "Meiotic recombination protein REC114",
  "gene": "UniProtKB:Q7Z4M0",
  "gene_symbol": "REC114",
  "term_id": "UNKNOWN:0003"
}